{
  "gene": "UniProtKB:P08133",
  "gene_symbol": "ANXA6",
  "term_id": "GO:0005886",
  "term_label": "plasma membrane",
  "gene_name": "Annexin A6"
}